{
  "term_id": "GO:0005879",
  "term_label": "axonemal microtubule",
  "gene": "UniProtKB:Q658L1",
  "gene_name": "Stabilizer of axonemal microtubules 2",
  "gene_symbol": "SAXO2"
}